{
  "gene_symbol": "TFRC",
  "gene_name": "Transferrin receptor protein 1",
  "gene": "UniProtKB:P02786",
  "term_label": "iron ion transport",
  "term_id": "GO:0006826"
}